{
  "gene_name": "Putative WAS protein family homolog 3",
  "gene_symbol": "WASH3P",
  "term_label": "retrograde transport, endosome to Golgi",
  "gene": "UniProtKB:C4AMC7",
  "term_id": "GO:0042147"
}